{
  "gene_symbol": "IGKC",
  "term_label": "immunoglobulin mediated immune response",
  "term_id": "GO:0016064",
  "gene_name": "Immunoglobulin kappa constant",
  "gene": "UniProtKB:P01834"
}